nucleoside monophosphate biosynthetic process [GO:0009124] (BP) Sources: GOC:go_curators, ISBN:0198506732 Definition: The chemical reactions and pathways resulting in the formation of a nucleoside monophosphate, a compound consisting of a nucleobase linked to a deoxyribose or ribose sugar esterified with phosphate on the sugar. Subtypes: purine nucleoside monophosphate biosynthetic process [GO:0009127], pyrimidine nucleoside monophosphate biosynthetic process [GO:0009130], ribonucleoside monophosphate biosynthetic process [GO:0009156], deoxyribonucleoside monophosphate biosynthetic process [GO:0009157] Relationships: is a type of GO:0009123; is a type of nucleoside phosphate biosynthetic process [GO:1901293] Also known as: nucleoside monophosphate anabolism, nucleoside monophosphate biosynthesis, nucleoside monophosphate formation, nucleoside monophosphate synthesis